{
  "gene_symbol": "DCDC2B",
  "gene_name": "Doublecortin domain-containing protein 2B",
  "gene": "UniProtKB:A2VCK2",
  "term_id": "UNKNOWN:0001",
  "term_label": "Unknown molecular function"
}